{
  "term_label": "Unknown molecular function",
  "term_id": "UNKNOWN:0001",
  "gene_symbol": "LACRT",
  "gene": "UniProtKB:Q9GZZ8",
  "gene_name": "Extracellular glycoprotein lacritin"
}